regulation of biological process [GO:0050789] (biological process) Relationships: is a type of biological regulation [GO:0065007]; RO_0002211 biological_process [GO:0008150] Definition: Any process that modulates the frequency, rate or extent of a biological process. Biological processes are regulated by many means; examples include the control of gene expression, protein modification or interaction with a protein or substrate molecule. Sources: GOC:ai, GOC:go_curators Subtypes: GO:0002682, regulation of signaling [GO:0023051], signaling [GO:0023052], regulation of cellular pH reduction [GO:0032847], GO:0032879, regulation of growth [GO:0040008], GO:0040012, regulation of circadian rhythm [GO:0042752], GO:0043903, modulation of formation of structure involved in a symbiotic process [GO:0044145], positive regulation of biological process [GO:0048518], GO:0048519, regulation of response to stimulus [GO:0048583], GO:0050792, GO:0050793, regulation of cellular process [GO:0050794], regulation of multicellular organismal process [GO:0051239], regulation of membrane repolarization [GO:0060306], GO:0097006, regulation of action potential [GO:0098900], GO:0120305, regulation of hemostasis [GO:1900046], regulation of membrane hyperpolarization [GO:1902630], GO:2000241 Also known as: regulation of physiological process